{
  "term_label": "Unknown cellular component",
  "term_id": "UNKNOWN:0003",
  "gene_name": "Annexin-2 receptor",
  "gene": "UniProtKB:Q3ZCQ2",
  "gene_symbol": "ANXA2R"
}